{
  "term_label": "neuron projection",
  "gene_symbol": "RIC3",
  "gene": "UniProtKB:Q7Z5B4",
  "term_id": "GO:0043005",
  "gene_name": "Protein RIC-3"
}